{
  "term_id": "UNKNOWN:0001",
  "term_label": "Unknown molecular function",
  "gene_name": "Lipoamide acyltransferase component of branched-chain alpha-keto acid dehydrogenase complex, mitochondrial",
  "gene_symbol": "DBT",
  "gene": "UniProtKB:P11182"
}